regulation of myeloid leukocyte mediated immunity [GO:0002886] (biological process) Subtypes: regulation of type III hypersensitivity [GO:0001803], GO:0002733, negative regulation of myeloid leukocyte mediated immunity [GO:0002887], positive regulation of myeloid leukocyte mediated immunity [GO:0002888], regulation of type II hypersensitivity [GO:0002892], regulation of mast cell degranulation [GO:0043304], regulation of eosinophil degranulation [GO:0043309], GO:0043313, regulation of neutrophil mediated cytotoxicity [GO:0070948], GO:1903581, regulation of microglial cell mediated cytotoxicity [GO:1904149] Relationships: is a type of GO:0002703; regulates myeloid leukocyte mediated immunity [GO:0002444] Sources: GOC:add Definition: Any process that modulates the frequency, rate, or extent of myeloid leukocyte mediated immunity.